{
  "term_id": "GO:0005666",
  "gene_name": "DNA-directed RNA polymerase III subunit RPC5",
  "term_label": "RNA polymerase III complex",
  "gene_symbol": "POLR3E",
  "gene": "UniProtKB:Q9NVU0"
}